postsynaptic endosome [GO:0098845] (cellular component) Relationships: is a type of endosome [GO:0005768]; is part of postsynapse [GO:0098794] References: PMID:20820847 Subtypes: postsynaptic recycling endosome [GO:0098837], postsynaptic early endosome [GO:0098842] Definition: An endosomal compartment that is part of the post-synapse. Only early and recycling endosomes are typically present in the postsynapse.